nuclear membrane biogenesis [GO:0101025] (biological process) Definition: The process in which a nuclear membrane is synthesized, aggregates, and bonds together. Sources: GOC:vw Relationships: is a type of membrane biogenesis [GO:0044091]; is part of nuclear membrane organization [GO:0071763] Subtypes: mitotic nuclear membrane biogenesis [GO:0101026]